NAD+ synthase activity [GO:0008795] (molecular function) Definition: Catalysis of the reaction: ATP + deamido-NAD+ + NH3 = AMP + diphosphate + NAD+. Also known as: NAD synthase (AMP-forming), NAD synthase activity, NAD synthetase activity, NAD(+) synthetase activity, NAD+ synthetase activity, deamido-NAD+:ammonia ligase (AMP-forming), diphosphopyridine nucleotide synthetase activity, nicotinamide adenine dinucleotide synthetase activity Relationships: is a type of acid-ammonia (or amide) ligase activity [GO:0016880] Sources: EC:6.3.1.5